{
  "gene": "UniProtKB:O14901",
  "term_label": "regulation of transcription by RNA polymerase II",
  "term_id": "GO:0006357",
  "gene_symbol": "KLF11",
  "gene_name": "Krueppel-like factor 11"
}